{
  "gene_name": "Bone morphogenetic protein 1",
  "gene": "UniProtKB:P13497",
  "gene_symbol": "BMP1",
  "term_label": "protein processing",
  "term_id": "GO:0016485"
}